{
  "gene": "UniProtKB:O15392",
  "term_label": "kinetochore",
  "gene_name": "Baculoviral IAP repeat-containing protein 5",
  "gene_symbol": "BIRC5",
  "term_id": "GO:0000776"
}